{
  "term_label": "extracellular space",
  "term_id": "GO:0005615",
  "gene": "UniProtKB:P04439",
  "gene_symbol": "HLA-A",
  "gene_name": "HLA class I histocompatibility antigen, A alpha chain"
}